{
  "gene": "UniProtKB:Q8N1I0",
  "term_id": "GO:0060326",
  "gene_name": "Dedicator of cytokinesis protein 4",
  "term_label": "cell chemotaxis",
  "gene_symbol": "DOCK4"
}